{
  "term_label": "Unknown molecular function",
  "gene_name": "Leucine-rich repeat-containing protein 31",
  "gene_symbol": "LRRC31",
  "term_id": "UNKNOWN:0001",
  "gene": "UniProtKB:Q6UY01"
}